{
  "gene": "UniProtKB:O14763",
  "term_id": "GO:0036462",
  "gene_name": "Tumor necrosis factor receptor superfamily member 10B",
  "gene_symbol": "TNFRSF10B",
  "term_label": "TRAIL-activated apoptotic signaling pathway"
}